{
  "term_id": "GO:0035804",
  "term_label": "structural constituent of egg coat",
  "gene_symbol": "ZP2",
  "gene": "UniProtKB:Q05996",
  "gene_name": "Zona pellucida sperm-binding protein 2"
}